{
  "gene_name": "U6 snRNA phosphodiesterase 1",
  "term_label": "U6 snRNA 3'-end processing",
  "gene_symbol": "USB1",
  "term_id": "GO:0034477",
  "gene": "UniProtKB:Q9BQ65"
}